{
  "term_id": "GO:0042383",
  "gene_name": "Synemin",
  "term_label": "sarcolemma",
  "gene_symbol": "SYNM",
  "gene": "UniProtKB:O15061"
}